{
  "term_label": "Unknown biological process",
  "gene_name": "BTB_POZ domain-containing protein KCTD3",
  "term_id": "UNKNOWN:0002",
  "gene": "UniProtKB:Q9Y597",
  "gene_symbol": "KCTD3"
}